{
  "gene_name": "Vomeronasal type-1 receptor 4",
  "term_id": "GO:0005550",
  "gene_symbol": "VN1R4",
  "gene": "UniProtKB:Q7Z5H5",
  "term_label": "pheromone binding"
}